lateral mesodermal cell fate specification [GO:0048377] (biological process) Relationships: is_a mesodermal cell fate specification [GO:0007501]; is part of GO:0048372 Also known as: lateral mesoderm cell fate specification, lateral plate mesoderm cell fate specification, lateral plate mesodermal cell fate specification Sources: GOC:jid Regulation: regulated by GO:0048378; positively regulated by positive regulation of lateral mesodermal cell fate specification [GO:0048379]; negatively regulated by negative regulation of lateral mesodermal cell fate specification [GO:0048380] Definition: The process in which a cell becomes capable of differentiating autonomously into a lateral mesoderm cell in an environment that is neutral with respect to the developmental pathway; upon specification, the cell fate can be reversed.